{
  "term_id": "GO:0050804",
  "gene_symbol": "GRIK2",
  "gene_name": "Glutamate receptor ionotropic, kainate 2",
  "gene": "UniProtKB:Q13002",
  "term_label": "modulation of chemical synaptic transmission"
}